{
  "term_id": "GO:0007186",
  "gene_name": "P2Y purinoceptor 4",
  "term_label": "G protein-coupled receptor signaling pathway",
  "gene_symbol": "P2RY4",
  "gene": "UniProtKB:P51582"
}